hydrogenase activity (NAD+, ferredoxin) [GO:0102220] (molecular function) Definition: Catalysis of the reaction: 2 dihydrogen + NAD + 2 an oxidized ferredoxin = NADH + 3 H+ + 2 a reduced ferredoxin. Relationships: is a type of GO:0016696 Sources: GOC:pz, RHEA:30279